{
  "gene": "UniProtKB:Q9NQZ7",
  "gene_name": "Ectonucleoside triphosphate diphosphohydrolase 7",
  "gene_symbol": "ENTPD7",
  "term_label": "UDP catabolic process",
  "term_id": "GO:0006256"
}